{
  "term_id": "GO:0005892",
  "term_label": "acetylcholine-gated channel complex",
  "gene": "UniProtKB:P17787",
  "gene_symbol": "CHRNB2",
  "gene_name": "Neuronal acetylcholine receptor subunit beta-2"
}